{
  "gene_symbol": "OTOF",
  "gene": "UniProtKB:Q9HC10",
  "gene_name": "Otoferlin",
  "term_id": "GO:0005509",
  "term_label": "calcium ion binding"
}